atrial cardiac muscle cell to AV node cell communication [GO:0086066] (biological process) Also known as: atrial cardiomyocyte to AV node cell communication, atrial cardiomyocyte to atrioventricular node cell communication Sources: GOC:BHF, GOC:mtg_cardiac_conduct_nov11 Definition: The process that mediates interactions between an atrial cardiomyocyte and its surroundings that contributes to the process of the atrial cardiomyocyte communicating with an AV node cell in cardiac conduction. Encompasses interactions such as signaling or attachment between one cell and another cell, between a cell and an extracellular matrix, or between a cell and any other aspect of its environment. Subtypes: atrial cardiac muscle cell to AV node cell signaling [GO:0086026], atrial cardiac muscle cell to AV node cell communication by electrical coupling [GO:0086044] Relationships: is_a GO:0086065